positive regulation of patulin biosynthetic process [GO:0140724] (biological process) Definition: Any process that increases the rate, frequency or extent of the chemical reactions and pathways resulting in the formation of patulin. References: PMID:25625822 Also known as: positive regulation of patulin anabolism, positive regulation of patulin formation, positive regulation of patulin synthesis Relationships: is a type of positive regulation of polyketide biosynthetic process [GO:1900734]; is_a positive regulation of alcohol biosynthetic process [GO:1902932]; positively regulates GO:0140723